mesenchymal cell migration involved in limb bud formation [GO:0035322] (BP) Relationships: is a type of GO:0090497; is part of GO:0090496 Definition: The orderly movement of a mesenchymal cell from one site to another that will contribute to the formation of a limb bud. Sources: GOC:dgh